{
  "term_label": "membrane",
  "term_id": "GO:0016020",
  "gene": "UniProtKB:Q9Y2W3",
  "gene_symbol": "SLC45A1",
  "gene_name": "Proton-associated sugar transporter A"
}